{
  "gene_name": "Uncharacterized protein C1orf185",
  "gene": "UniProtKB:Q5T7R7",
  "term_label": "Unknown cellular component",
  "gene_symbol": "C1orf185",
  "term_id": "UNKNOWN:0003"
}